{
  "term_label": "nucleus",
  "term_id": "GO:0005634",
  "gene_symbol": "MEIS3",
  "gene": "UniProtKB:Q99687",
  "gene_name": "Homeobox protein Meis3"
}